{
  "term_id": "GO:0097157",
  "gene_name": "Pre-mRNA-processing-splicing factor 8",
  "gene": "UniProtKB:Q6P2Q9",
  "term_label": "pre-mRNA intronic binding",
  "gene_symbol": "PRPF8"
}